monomethyl-sulfatase activity [GO:0050106] (molecular function) Relationships: is a type of sulfuric ester hydrolase activity [GO:0008484] Sources: EC:3.1.6.16, RHEA:14221 Also known as: monomethyl-sulphatase activity, monomethyl-sulfate sulfohydrolase activity Definition: Catalysis of the reaction: H2O + monomethyl sulfate = H+ + methanol + sulfate.